{
  "gene": "UniProtKB:O43399",
  "gene_name": "Tumor protein D54",
  "gene_symbol": "TPD52L2",
  "term_label": "Unknown biological process",
  "term_id": "UNKNOWN:0002"
}